{
  "gene_name": "Paraneoplastic antigen Ma6E",
  "gene": "UniProtKB:A0A0J9YXQ4",
  "term_label": "Unknown cellular component",
  "term_id": "UNKNOWN:0003",
  "gene_symbol": "PNMA6E"
}